{
  "term_label": "tubulin binding",
  "gene_symbol": "RITA1",
  "term_id": "GO:0015631",
  "gene_name": "RBPJ-interacting and tubulin-associated protein 1",
  "gene": "UniProtKB:Q96K30"
}